{
  "term_label": "cytoplasm",
  "gene_name": "Kinesin-like protein KIF2A",
  "term_id": "GO:0005737",
  "gene_symbol": "KIF2A",
  "gene": "UniProtKB:O00139"
}